venom-mediated perturbation of hemostasis [GO:0044483] (biological process) Subtypes: venom-mediated hemorrhage [GO:0044358], GO:0044468, venom-mediated suppression of platelet aggregation [GO:0044477], venom-mediated fibrinolysis [GO:0044484], venom-mediated depletion of circulating fibrinogen [GO:0044536], venom-mediated suppression of fibrinolysis [GO:0140099] Sources: GOC:fj, GOC:jl Relationships: is a type of venom-mediated perturbation of blood circulation [GO:0140134] Definition: A process in which an organism alters or subverts hemostasis in another organism via the action of a venom. Hemostasis is the mechanism that leads to cessation of bleeding from a blood vessel. Also known as: envenomation perturbing hemostasis, envenomation resulting in impairment of hemostasis in another organism, envenomation resulting in impairment of hemostasis in other organism, envenomation resulting in negative regulation of hemostasis in other organism, envenomation, impairing hemostasis in other organism